{
  "gene_symbol": "JRKL",
  "term_id": "GO:0005634",
  "gene": "UniProtKB:Q9Y4A0",
  "term_label": "nucleus",
  "gene_name": "Jerky protein homolog-like"
}